{
  "gene_symbol": "TBC1D3D",
  "gene_name": "TBC1 domain family member 3D",
  "term_id": "UNKNOWN:0002",
  "term_label": "Unknown biological process",
  "gene": "UniProtKB:A0A087WVF3"
}